{
  "gene_name": "Heat shock transcription factor, Y-linked",
  "gene_symbol": "HSFY2",
  "term_label": "Unknown biological process",
  "term_id": "UNKNOWN:0002",
  "gene": "UniProtKB:Q96LI6"
}